regulation of mitochondrion organization [GO:0010821] (biological process) Subtypes: GO:0010635, GO:0090140, regulation of release of cytochrome c from mitochondria [GO:0090199], regulation of mitochondrial outer membrane permeabilization involved in apoptotic signaling pathway [GO:1901028], positive regulation of mitochondrial DNA metabolic process [GO:1901860], regulation of protein insertion into mitochondrial outer membrane [GO:1903636], regulation of cristae formation [GO:1903850] Relationships: is a type of regulation of organelle organization [GO:0033043]; regulates mitochondrion organization [GO:0007005] Also known as: regulation of mitochondrion organisation Definition: Any process that modulates the frequency, rate or extent of a process involved in the formation, arrangement of constituent parts, or disassembly of a mitochondrion. Sources: GOC:dph, GOC:tb